Swi5-Swi2 complex [GO:0034974] (cellular component) Relationships: is a type of nuclear protein-containing complex [GO:0140513]; is part of GO:0000228; is part of GO:0000785 Also known as: Swi5 complex References: PMID:14663140 Note: Note that this term refers to Schizosaccharomyces pombe Swi5 and Swi2, which should not be confused with the unrelated Saccharomyces Swi5p and Swi2p. Definition: A protein complex involved that contains proteins known in Schizosaccharomyces as Swi5 monomers and Swi2, and is involved in mating type switching.